{
  "gene": "UniProtKB:Q96PN6",
  "term_label": "adenylate cyclase activity",
  "term_id": "GO:0004016",
  "gene_symbol": "ADCY10",
  "gene_name": "Adenylate cyclase type 10"
}